{
  "term_label": "Unknown biological process",
  "gene_name": "Bombesin receptor-activated protein C6orf89",
  "gene": "UniProtKB:Q6UWU4",
  "term_id": "UNKNOWN:0002",
  "gene_symbol": "C6orf89"
}